{
  "gene": "UniProtKB:Q7L5Y9",
  "gene_name": "E3 ubiquitin-protein transferase MAEA",
  "term_id": "GO:0005634",
  "gene_symbol": "MAEA",
  "term_label": "nucleus"
}